{
  "term_id": "GO:0005886",
  "gene_symbol": "CFAP95",
  "term_label": "plasma membrane",
  "gene": "UniProtKB:Q5VTT2",
  "gene_name": "Cilia- and flagella-associated protein 95"
}